{
  "gene": "UniProtKB:A6NLC8",
  "term_label": "RNA polymerase II general transcription initiation factor activity",
  "gene_symbol": "TAF11L2",
  "term_id": "GO:0016251",
  "gene_name": "TATA-box binding protein associated factor 11 like protein 2"
}